{
  "term_id": "UNKNOWN:0001",
  "gene": "UniProtKB:Q330K2",
  "gene_symbol": "NDUFAF6",
  "gene_name": "NADH dehydrogenase (ubiquinone) complex I, assembly factor 6",
  "term_label": "Unknown molecular function"
}